{
  "gene": "UniProtKB:Q8TD16",
  "term_id": "GO:0005829",
  "term_label": "cytosol",
  "gene_name": "Protein bicaudal D homolog 2",
  "gene_symbol": "BICD2"
}